regulation of L-leucine import across plasma membrane [GO:1905532] (biological process) Relationships: is a type of GO:0010958; is a type of GO:0032890; regulates L-leucine import across plasma membrane [GO:1903801] Also known as: regulation of L-leucine import into cell Definition: Any process that modulates the frequency, rate or extent of L-leucine import across plasma membrane. Subtypes: negative regulation of L-leucine import across plasma membrane [GO:1905533], positive regulation of L-leucine import across plasma membrane [GO:1905534] References: PMID:10467003 Sources: GOC:TermGenie, GO_REF:0000058